{
  "gene_symbol": "FEM1A",
  "gene_name": "Protein fem-1 homolog A",
  "term_label": "negative regulation of inflammatory response",
  "term_id": "GO:0050728",
  "gene": "UniProtKB:Q9BSK4"
}